{
  "gene": "UniProtKB:Q9ULD0",
  "gene_symbol": "OGDHL",
  "gene_name": "2-oxoglutarate dehydrogenase-like, mitochondrial",
  "term_id": "GO:0005739",
  "term_label": "mitochondrion"
}